periarbuscular membrane [GO:0085042] (cellular component) Sources: GOC:pamgo_curators Relationships: is a type of GO:0033644 Definition: A host-derived membrane surrounding the symbiont arbuscule during symbiosis. Note: See also: arbuscule ; GO:0085041.